{
  "term_label": "aspartic-type endopeptidase activity",
  "gene": "UniProtKB:P12273",
  "gene_name": "Prolactin-inducible protein",
  "gene_symbol": "PIP",
  "term_id": "GO:0004190"
}